hyaluronoglucuronidase activity [GO:0033906] (molecular function) Definition: Catalysis of the random hydrolysis of 1,3-linkages between beta-D-glucuronate and N-acetyl-D-glucosamine residues in hyaluronate. Relationships: is a type of glucuronidase activity [GO:0046574] Also known as: hyaluronidase activity, glucuronoglucosaminoglycan hyaluronate lyase activity, hyaluronate 3-glycanohydrolase activity, orgelase activity Sources: EC:3.2.1.36